{
  "gene_name": "Protein RFT1 homolog",
  "gene": "UniProtKB:Q96AA3",
  "term_label": "endoplasmic reticulum membrane",
  "term_id": "GO:0005789",
  "gene_symbol": "RFT1"
}